negative regulation of protein refolding [GO:0061084] (biological process) Relationships: is a type of regulation of protein refolding [GO:0061083]; is a type of negative regulation of protein folding [GO:1903333]; negatively regulates protein refolding [GO:0042026] Definition: Any process that decreases the rate, frequency, or extent of protein refolding. Protein refolding is the process carried out by a cell that restores the biological activity of an unfolded or misfolded protein, using helper proteins such as chaperones. Sources: GOC:BHF, GOC:dph, GOC:tb